negative regulation of cerebellar neuron development [GO:1905080] (biological process) Relationships: is a type of negative regulation of cell development [GO:0010721]; is a type of negative regulation of neuron differentiation [GO:0045665]; is a type of regulation of cerebellar neuron development [GO:1905079]; negatively regulates cerebellar neuron development [GO:0098749] Also known as: down regulation of cerebellar neuron development, down-regulation of cerebellar neuron development, downregulation of cerebellar neuron development, inhibition of cerebellar neuron development Definition: Any process that stops, prevents or reduces the frequency, rate or extent of cerebellar neuron development. References: PMID:26609159 Sources: GOC:TermGenie, GO_REF:0000058